{
  "term_id": "GO:0005604",
  "gene_symbol": "LAMB3",
  "term_label": "basement membrane",
  "gene": "UniProtKB:Q13751",
  "gene_name": "Laminin subunit beta-3"
}